{
  "term_label": "Unknown molecular function",
  "gene_symbol": "FAM234A",
  "term_id": "UNKNOWN:0001",
  "gene_name": "Protein FAM234A",
  "gene": "UniProtKB:Q9H0X4"
}